tRNA (adenine(37)-C2)-methyltransferase activity [GO:0002935] (molecular function) References: PMID:22891362 Sources: RHEA:43332 Relationships: is a type of C-methyltransferase activity [GO:0008169]; is a type of tRNA (adenine) methyltransferase activity [GO:0016426] Definition: Catalysis of the reaction: adenosine37 in tRNA + 2 reduced [2Fe-2S]-[ferredoxin] + 2 S-adenosyl-L-methionine = 2-methyladenosine37 in tRNA + 5'-deoxyadenosine + L-methionine + 2 oxidized [2Fe-2S]-[ferredoxin] + S-adenosyl-L-homocysteine. Also known as: tRNA (adenine(37)-C(2))-methyltransferase activity, tRNA (adenosine(37)-C2-)-methyltransferase activity